{
  "term_label": "Unknown biological process",
  "term_id": "UNKNOWN:0002",
  "gene_symbol": "GARNL3",
  "gene_name": "GTPase-activating Rap_Ran-GAP domain-like protein 3",
  "gene": "UniProtKB:Q5VVW2"
}